phosphate ion uniporter activity [GO:0140787] (molecular function) Relationships: is a type of GO:0005315; is a type of membrane potential driven uniporter activity [GO:0022810] Definition: Catalysis of the active transport of a phosphate ion across a membrane by a mechanism involving conformational change, where energy for active transport is derived from membrane potential if the solute is charged. References: PMID:29642010